regulation of adenylate cyclase-activating glucose-activated G protein-coupled receptor signaling pathway [GO:0110033] (biological process) Also known as: regulation of adenylate cyclase-activating glucose-activated G-protein coupled receptor signaling pathway Relationships: is a type of regulation of adenylate cyclase-activating G protein-coupled receptor signaling pathway [GO:0106070]; is a type of regulation of glucose mediated signaling pathway [GO:1902659]; regulates GO:0010619 Subtypes: negative regulation of adenylate cyclase-activating glucose-activated G protein-coupled receptor signaling pathway [GO:0110034] Definition: Any process that modulates the frequency, rate or extent of the adenylate cyclase-activating glucose-activated G protein-coupled receptor signaling pathway, the series of molecular signals generated as a consequence of glucose binding to a G protein-coupled receptor, where the pathway proceeds with activation of adenylyl cyclase and a subsequent increase in the concentration of cyclic AMP (cAMP). References: PMID:24297439 Sources: GOC:al